{
  "gene_symbol": "TIMP3",
  "gene": "UniProtKB:P35625",
  "term_label": "metalloendopeptidase inhibitor activity",
  "gene_name": "Metalloproteinase inhibitor 3",
  "term_id": "GO:0008191"
}